{
  "term_label": "Unknown molecular function",
  "term_id": "UNKNOWN:0001",
  "gene_name": "Ig-like domain-containing protein (Fragment)",
  "gene_symbol": "A0A0G2JRQ6",
  "gene": "UniProtKB:A0A0G2JRQ6"
}